{
  "gene_name": "Cathepsin L2",
  "term_label": "lysosome",
  "gene": "UniProtKB:O60911",
  "term_id": "GO:0005764",
  "gene_symbol": "CTSV"
}